{
  "term_id": "UNKNOWN:0001",
  "term_label": "Unknown molecular function",
  "gene_name": "Synaptic vesicle membrane protein VAT-1 homolog",
  "gene_symbol": "VAT1",
  "gene": "UniProtKB:Q99536"
}